{
  "gene_symbol": "NAA16",
  "term_id": "GO:0010698",
  "gene_name": "N-alpha-acetyltransferase 16, NatA auxiliary subunit",
  "term_label": "acetyltransferase activator activity",
  "gene": "UniProtKB:Q6N069"
}